{
  "gene_symbol": "FSHB",
  "gene_name": "Follitropin subunit beta",
  "term_label": "follicle-stimulating hormone activity",
  "term_id": "GO:0016913",
  "gene": "UniProtKB:P01225"
}